{
  "gene_name": "Alpha-1,3-mannosyl-glycoprotein 4-beta-N-acetylglucosaminyltransferase A",
  "gene": "UniProtKB:Q9UM21",
  "gene_symbol": "MGAT4A",
  "term_id": "GO:0008375",
  "term_label": "acetylglucosaminyltransferase activity"
}